{
  "gene_name": "Gamma-aminobutyric acid receptor subunit epsilon",
  "gene_symbol": "GABRE",
  "term_id": "GO:1902711",
  "gene": "UniProtKB:P78334",
  "term_label": "GABA-A receptor complex"
}